histone H1-4S35 kinase activity [GO:0140198] (molecular function) References: PMID:21852232 Definition: Catalysis of the reaction: histone H1-4-serine (position 35) + ATP = histone H1-4-phosphoserine (position 35) + ADP. Relationships: is a type of protein serine/threonine kinase activity [GO:0004674]; is a type of GO:0140190